{
  "term_label": "polyubiquitin modification-dependent protein binding",
  "gene_symbol": "PSMD4",
  "term_id": "GO:0031593",
  "gene_name": "26S proteasome non-ATPase regulatory subunit 4",
  "gene": "UniProtKB:P55036"
}